{
  "gene_name": "Interferon alpha-21",
  "gene": "UniProtKB:P01568",
  "gene_symbol": "IFNA21",
  "term_label": "response to exogenous dsRNA",
  "term_id": "GO:0043330"
}